plant-type cell wall assembly [GO:0071668] (biological process) Definition: The aggregation, arrangement and bonding together of a set of components to form a cellulose- and pectin-containing cell wall. Also known as: plant cell wall assembly Relationships: is a type of GO:0009664; is a type of cell wall assembly [GO:0070726]; is part of plant-type cell wall biogenesis [GO:0009832] Sources: GOC:mah